{
  "term_id": "GO:0005047",
  "gene": "UniProtKB:Q96Q80",
  "term_label": "signal recognition particle binding",
  "gene_symbol": "DERL3",
  "gene_name": "Derlin-3"
}